L-ascorbic acid transmembrane transporter activity [GO:0015229] (molecular function) Definition: Enables the transfer of L-ascorbate from one side of a membrane to the other. L-ascorbate, (2R)-2-[(1S)-1,2-dihydroxyethyl]-4-hydroxy-5-oxo-2,5-dihydrofuran-3-olate, is vitamin C and has co-factor and anti-oxidant activities in many species. Sources: ISBN:0198506732 Also known as: L-ascorbate transporter activity, vitamin C transporter activity Relationships: is a type of monosaccharide transmembrane transporter activity [GO:0015145]; is_a carboxylic acid transmembrane transporter activity [GO:0046943]; is a type of vitamin transmembrane transporter activity [GO:0090482]; is part of L-ascorbic acid transmembrane transport [GO:0015882]